{
  "gene_symbol": "SPP2",
  "term_label": "Unknown molecular function",
  "term_id": "UNKNOWN:0001",
  "gene": "UniProtKB:Q13103",
  "gene_name": "Secreted phosphoprotein 24"
}